{
  "term_id": "GO:0015629",
  "term_label": "actin cytoskeleton",
  "gene": "UniProtKB:Q5JWF8",
  "gene_name": "Actin-like protein 10",
  "gene_symbol": "ACTL10"
}